{
  "term_label": "cytoplasm",
  "term_id": "GO:0005737",
  "gene": "UniProtKB:Q9P0R6",
  "gene_symbol": "GSKIP",
  "gene_name": "GSK3B-interacting protein"
}